subpallium neuron fate commitment [GO:0060163] (BP) Also known as: subpallium neuronal precursor fate commitment Sources: GOC:dph Relationships: is a type of neuron fate commitment [GO:0048663]; is part of GO:0021544 Definition: The process in which in the subpallium, the developmental fate of a cell becomes restricted such that it will develop into a neuron. The subpallium is the base region of the telencephalon.